{
  "gene_name": "Cell adhesion molecule DSCAML1",
  "term_label": "axon",
  "gene": "UniProtKB:Q8TD84",
  "term_id": "GO:0030424",
  "gene_symbol": "DSCAML1"
}